12-hydroxydihydrochelirubine 12-O-methyltransferase activity [GO:0030780] (molecular function) Definition: Catalysis of the reaction: 12-hydroxydihydrochelirubine + S-adenosyl-L-methionine(1+) = S-adenosyl-L-homocysteine + dihydromacarpine + H+. Relationships: is a type of S-adenosylmethionine-dependent methyltransferase activity [GO:0008757] Sources: EC:2.1.1.120, RHEA:21092 Also known as: S-adenosyl-L-methionine:12-hydroxydihydrochelirubine 12-O-methyltransferase activity